negative regulation of nuclear-transcribed mRNA poly(A) tail shortening [GO:0060212] (biological process) Relationships: is a type of GO:0060211; is a type of negative regulation of nuclear-transcribed mRNA catabolic process, deadenylation-dependent decay [GO:1900152]; negatively regulates nuclear-transcribed mRNA poly(A) tail shortening [GO:0000289] Sources: GOC:dph, GOC:tb Definition: Any process that decreases the frequency, rate or extent of poly(A) tail shortening of a nuclear-transcribed mRNA. Poly(A) tail shortening is the decrease in length of the poly(A) tail of an mRNA from full length to an oligo(A) length. Also known as: negative regulation of 3' to 5' mRNA deadenylation, negative regulation of mRNA deadenylation, negative regulation of nuclear mRNA poly(A) tail shortening